senescence-associated heterochromatin focus [GO:0035985] (cellular component) References: PMID:15621527, PMID:21248468 Sources: GOC:yaf Also known as: SAHF, senescence-associated heterochromatin foci Definition: A transcriptionally-silent heterochromatin structure present in senescent cells. Contains the condensed chromatin of one chromosome and is enriched for histone modifications. Thought to repress expression of proliferation-promoting genes. Relationships: is a type of heterochromatin [GO:0000792]